{
  "gene_name": "cAMP-dependent protein kinase type I-alpha regulatory subunit",
  "term_id": "GO:0005952",
  "term_label": "cAMP-dependent protein kinase complex",
  "gene": "UniProtKB:P10644",
  "gene_symbol": "PRKAR1A"
}